{
  "term_label": "Unknown molecular function",
  "gene": "UniProtKB:A0A075B6V0",
  "term_id": "UNKNOWN:0001",
  "gene_name": "T cell receptor alpha joining 16 (Fragment)",
  "gene_symbol": "TRAJ16"
}